{
  "gene_name": "Cyclin-dependent kinase-like 2",
  "gene_symbol": "CDKL2",
  "term_label": "protein serine/threonine kinase activity",
  "term_id": "GO:0004674",
  "gene": "UniProtKB:Q92772"
}